BH3 domain binding [GO:0051434] (molecular function) Relationships: is a type of BH domain binding [GO:0051400]; is_a death domain binding [GO:0070513] Definition: Binding to a BH3 protein domain, present in Bcl-2 family members. The BH3 domain is a potent death domain and has an important role in protein-protein interactions and in cell death. References: PMID:11048732, PMID:12133724, PMID:9020082, PMID:9704409 Sources: Prosite:PS01259